{
  "term_id": "GO:0005085",
  "gene_name": "Protein transport protein Sec61 subunit beta",
  "gene_symbol": "SEC61B",
  "gene": "UniProtKB:P60468",
  "term_label": "guanyl-nucleotide exchange factor activity"
}